glyceraldehyde-3-phosphate dehydrogenase (NAD+) (non-phosphorylating) activity [GO:0043878] (molecular function) Also known as: NAD+-dependent glyceraldehyde-3-phosphate dehydrogenase activity, glyceraldehyde-3-phosphate dehydrogenase (NAD) (non-phosphorylating) activity, glyceraldehyde-3-phosphate dehydrogenase (NAD) activity, non-phosphorylating glyceraldehyde-3-phosphate dehydrogenase (NAD) Definition: Catalysis of the reaction: D-glyceraldehyde 3-phosphate + NAD+ + H2O = 3-phospho-D-glycerate + NADH + H+. References: PMID:9497334 Relationships: is a type of GO:0120533